{
  "gene": "UniProtKB:Q12860",
  "gene_name": "Contactin-1",
  "term_id": "GO:0098609",
  "term_label": "cell-cell adhesion",
  "gene_symbol": "CNTN1"
}